starch grain [GO:0043036] (cellular component) Definition: Plant storage body for amylose and amylopectin, 1-100um in diameter. Also contains small amounts of enzymes, amino acids, lipids and nucleic acids. The shape of the grain varies widely amongst species, but is often spherical or disk-shaped. Subtypes: amyloplast starch grain [GO:0009568], chloroplast starch grain [GO:0009569] Also known as: starch granule Relationships: is a type of cellular anatomical structure [GO:0110165]; is part of plastid [GO:0009536] References: PMID:11217978 Sources: GOC:jl